acetolactate synthase activity [GO:0003984] (molecular function) Regulation: regulated by GO:1990610 Definition: Catalysis of the reaction: H+ + 2 pyruvate = (2S)-2-acetolactate + CO2. Can also convert 2-oxobutanoate and pyruvate to (S)-2-ethyl-2-hydroxy-3-oxobutanoate. Relationships: is a type of GO:0016744 Sources: EC:2.2.1.6 Also known as: acetohydroxy acid synthetase activity, acetohydroxyacid synthase activity, acetolactate pyruvate-lyase (carboxylating) activity, acetolactic synthetase activity, alpha-acetohydroxy acid synthetase activity, alpha-acetohydroxyacid synthase activity, alpha-acetolactate synthase activity, alpha-acetolactate synthetase activity, pyruvate:pyruvate acetaldehydetransferase (decarboxylating)